{
  "term_id": "UNKNOWN:0002",
  "gene_symbol": "XPNPEP1",
  "term_label": "Unknown biological process",
  "gene": "UniProtKB:Q9NQW7",
  "gene_name": "Xaa-Pro aminopeptidase 1"
}